{
  "term_id": "GO:0000049",
  "gene_name": "tRNA methyltransferase 10 homolog B",
  "gene_symbol": "TRMT10B",
  "term_label": "tRNA binding",
  "gene": "UniProtKB:Q6PF06"
}